positive regulation of type IIa hypersensitivity [GO:0001798] (BP) Relationships: is a type of regulation of type IIa hypersensitivity [GO:0001796]; is a type of GO:0002894; positively regulates type IIa hypersensitivity [GO:0001794] Definition: Any process that activates or increases the frequency, rate or extent of type IIa hypersensitivity, a type of inflammatory response. Also known as: up regulation of type IIa hypersensitivity, up-regulation of type IIa hypersensitivity, upregulation of type IIa hypersensitivity, activation of type IIa hypersensitivity, stimulation of type IIa hypersensitivity Subtypes: GO:0001815 Sources: GOC:add, ISBN:0781735149